{
  "gene": "UniProtKB:P51864",
  "gene_name": "Putative teratocarcinoma-derived growth factor 3",
  "term_id": "GO:0038100",
  "term_label": "nodal binding",
  "gene_symbol": "CRIPTO3"
}